horsetail-astral microtubule organization [GO:0032118] (biological process) Also known as: horsetail-astral microtubule array organization, horsetail-astral microtubule organisation, horsetail-astral microtubule organization and biogenesis Sources: GOC:mah Relationships: is a type of microtubule cytoskeleton organization [GO:0000226]; is a type of meiotic cell cycle process [GO:1903046]; is part of GO:0030989 Definition: A process that is carried out at the cellular level which results in the assembly, arrangement of constituent parts, or disassembly of the horsetail-astral array, a structure of astral microtubules that emanates from the spindle pole body during meiosis.